{
  "term_id": "GO:0001917",
  "term_label": "photoreceptor inner segment",
  "gene_name": "Coiled-coil domain-containing protein 66",
  "gene": "UniProtKB:A2RUB6",
  "gene_symbol": "CCDC66"
}